positive regulation of vein smooth muscle contraction [GO:0062087] (biological process) Relationships: is a type of regulation of vein smooth muscle contraction [GO:0062086]; is a type of positive regulation of vascular associated smooth muscle contraction [GO:1904695]; positively regulates vein smooth muscle contraction [GO:0014826] References: PMID:8428203 Definition: Any process that increases the frequency, rate or extent of vein smooth muscle contraction.